{
  "gene": "UniProtKB:Q9HD47",
  "gene_symbol": "RANGRF",
  "gene_name": "Ran guanine nucleotide release factor",
  "term_label": "transmembrane transporter binding",
  "term_id": "GO:0044325"
}